{
  "gene": "UniProtKB:O60462",
  "term_label": "plasma membrane",
  "term_id": "GO:0005886",
  "gene_name": "Neuropilin-2",
  "gene_symbol": "NRP2"
}